{
  "gene_name": "Lysophospholipid acyltransferase LPCAT4",
  "gene_symbol": "LPCAT4",
  "term_label": "Unknown biological process",
  "term_id": "UNKNOWN:0002",
  "gene": "UniProtKB:Q643R3"
}